{
  "gene_name": "F-box only protein 46",
  "term_id": "UNKNOWN:0002",
  "gene_symbol": "FBXO46",
  "gene": "UniProtKB:Q6PJ61",
  "term_label": "Unknown biological process"
}